positive regulation of intracellular lipid transport [GO:0032379] (biological process) Subtypes: GO:0032382 Also known as: up regulation of intracellular lipid transport, up-regulation of intracellular lipid transport, upregulation of intracellular lipid transport, activation of intracellular lipid transport, stimulation of intracellular lipid transport Relationships: is a type of GO:0032370; is a type of regulation of intracellular lipid transport [GO:0032377]; is a type of GO:0032388; positively regulates GO:0032365 Definition: Any process that activates or increases the frequency, rate or extent of the directed movement of lipids within cells. Sources: GOC:mah